oligosaccharide binding [GO:0070492] (molecular function) Relationships: is a type of carbohydrate binding [GO:0030246] Sources: GOC:mah Definition: Binding to an oligosaccharide, a molecule with between two and (about) 20 monosaccharide residues connected by glycosidic linkages. Subtypes: GO:0044584, cellotetraose binding [GO:0044586], cellopentaose binding [GO:0044587], laminaribiose binding [GO:0044588], GO:0048030, trisaccharide binding [GO:0048031], cellooligosaccharide binding [GO:2001064], maltoheptaose binding [GO:2001071], cyclodextrin binding [GO:2001073]